{
  "gene_symbol": "WRN",
  "term_label": "chromosome",
  "term_id": "GO:0005694",
  "gene_name": "Bifunctional 3'-5' exonuclease_ATP-dependent helicase WRN",
  "gene": "UniProtKB:Q14191"
}